{
  "gene_name": "General transcription factor II-I",
  "gene": "UniProtKB:P78347",
  "term_label": "Unknown biological process",
  "gene_symbol": "GTF2I",
  "term_id": "UNKNOWN:0002"
}